{
  "gene_symbol": "BRCC3",
  "gene": "UniProtKB:P46736",
  "term_id": "GO:0006302",
  "gene_name": "Lys-63-specific deubiquitinase BRCC36",
  "term_label": "double-strand break repair"
}